{
  "term_id": "UNKNOWN:0001",
  "gene_name": "Mediator of RNA polymerase II transcription subunit 7",
  "gene_symbol": "MED7",
  "gene": "UniProtKB:O43513",
  "term_label": "Unknown molecular function"
}